{
  "gene_name": "CTD small phosphatase-like protein",
  "gene_symbol": "CTDSPL",
  "term_label": "Unknown cellular component",
  "term_id": "UNKNOWN:0003",
  "gene": "UniProtKB:O15194"
}